{
  "gene_symbol": "ARID4A",
  "term_id": "GO:0006357",
  "gene": "UniProtKB:P29374",
  "term_label": "regulation of transcription by RNA polymerase II",
  "gene_name": "AT-rich interactive domain-containing protein 4A"
}